thiazole metabolic process [GO:0052838] (biological process) Definition: The chemical reactions and pathways involving thiazole, a five-membered heterocyclic ring structure containing a sulfur in the 1-position and a nitrogen in the 3-position. Sources: GOC:curators Also known as: thiazole metabolism Relationships: is a type of sulfur compound metabolic process [GO:0006790] Subtypes: thiazole biosynthetic process [GO:0052837]